negative regulation of MyD88-independent toll-like receptor signaling pathway [GO:0034128] (biological process) Relationships: is a type of GO:0034122; is a type of regulation of MyD88-independent toll-like receptor signaling pathway [GO:0034127]; negatively regulates GO:0002756 References: PMID:16551253, PMID:17328678 Sources: GOC:add Definition: Any process that stops, prevents, or reduces the frequency, rate, or extent of MyD88-independent toll-like receptor signaling pathway. Also known as: negative regulation of MyD88-independent TLR signaling pathway, negative regulation of MyD88-independent toll-like receptor signalling pathway